{
  "gene_symbol": "PMS2P2",
  "term_label": "Unknown biological process",
  "term_id": "UNKNOWN:0002",
  "gene": "UniProtKB:O95744",
  "gene_name": "Putative postmeiotic segregation increased 2-like protein 2"
}